{
  "gene_name": "Eukaryotic translation initiation factor 3 subunit F",
  "term_label": "translational initiation",
  "gene": "UniProtKB:O00303",
  "term_id": "GO:0006413",
  "gene_symbol": "EIF3F"
}